regulation of cell budding [GO:0007116] (biological process) Relationships: is a type of regulation of cell division [GO:0051302]; is a type of regulation of asexual reproduction [GO:1903664]; regulates cell budding [GO:0007114] Subtypes: GO:0045781, positive regulation of cell budding [GO:0045782] Sources: GOC:mah Definition: Any process that modulates the frequency, rate or extent of the formation and growth of cell buds. Also known as: regulation of budding